{
  "gene": "UniProtKB:Q6UWX4",
  "gene_symbol": "HHIPL2",
  "gene_name": "HHIP-like protein 2",
  "term_id": "UNKNOWN:0001",
  "term_label": "Unknown molecular function"
}